{
  "gene_symbol": "FHAD1",
  "gene": "UniProtKB:B1AJZ9",
  "term_label": "Unknown biological process",
  "term_id": "UNKNOWN:0002",
  "gene_name": "Forkhead-associated domain-containing protein 1"
}